G protein-coupled estrogen receptor activity [GO:0038054] (molecular function) Also known as: estrogen receptor activity, G-protein coupled estrogen receptor activity Relationships: is a type of G protein-coupled receptor activity [GO:0004930] References: PMID:17379646, PMID:20960099 Sources: GOC:signaling Definition: Combining with estrogen and transmitting the signal across the membrane by activating an associated G-protein; promotes the exchange of GDP for GTP on the alpha subunit of a heterotrimeric G-protein complex.